2-isopropylmalate(2-) transmembrane transport [GO:1902357] (biological process) Definition: The process in which 2-isopropylmalate(2-) is transported across a membrane. Relationships: is a type of isopropylmalate transport [GO:0034659]; is a type of carboxylic acid transmembrane transport [GO:1905039] References: PMID:18682385 Sources: GOC:TermGenie, GOC:dph, GOC:vw Subtypes: mitochondrial isopropylmalate transmembrane transport [GO:1990556]